{
  "gene": "UniProtKB:Q8NFL0",
  "term_label": "Golgi membrane",
  "term_id": "GO:0000139",
  "gene_symbol": "B3GNT7",
  "gene_name": "UDP-GlcNAc:betaGal beta-1,3-N-acetylglucosaminyltransferase 7"
}